{
  "gene": "UniProtKB:Q9BYQ9",
  "gene_symbol": "KRTAP4-8",
  "gene_name": "Keratin-associated protein 4-8",
  "term_label": "Unknown molecular function",
  "term_id": "UNKNOWN:0001"
}